{
  "term_id": "GO:0032956",
  "term_label": "regulation of actin cytoskeleton organization",
  "gene_name": "Rho-related BTB domain-containing protein 2",
  "gene_symbol": "RHOBTB2",
  "gene": "UniProtKB:Q9BYZ6"
}